{
  "term_label": "actin filament binding",
  "gene": "UniProtKB:Q13402",
  "term_id": "GO:0051015",
  "gene_name": "Unconventional myosin-VIIa",
  "gene_symbol": "MYO7A"
}